{
  "term_label": "Unknown cellular component",
  "gene": "UniProtKB:Q5T0Z8",
  "term_id": "UNKNOWN:0003",
  "gene_name": "Uncharacterized protein C6orf132",
  "gene_symbol": "C6orf132"
}